{
  "term_id": "GO:0017128",
  "gene_name": "Phospholipid scramblase 1",
  "term_label": "phospholipid scramblase activity",
  "gene_symbol": "PLSCR1",
  "gene": "UniProtKB:O15162"
}